{
  "term_id": "UNKNOWN:0002",
  "gene_symbol": "DCAF8",
  "gene": "UniProtKB:Q5TAQ9",
  "gene_name": "DDB1- and CUL4-associated factor 8",
  "term_label": "Unknown biological process"
}